positive regulation of maintenance of mitotic sister chromatid cohesion [GO:0034184] (biological process) Definition: Any process that increases the extent to which the association between sister chromatids of a replicated chromosome is maintained during a mitotic cell cycle. Sources: GOC:mah, GOC:vw Relationships: is a type of GO:0034093; is a type of regulation of maintenance of mitotic sister chromatid cohesion [GO:0034182]; positively regulates maintenance of mitotic sister chromatid cohesion [GO:0034088] Subtypes: positive regulation of maintenance of mitotic sister chromatid cohesion, telomeric [GO:1904909], positive regulation of maintenance of mitotic sister chromatid cohesion, arms [GO:2000717], positive regulation of maintenance of mitotic sister chromatid cohesion, centromeric [GO:2000720]